costunolide 3beta-hydroxylase activity [GO:0102628] (molecular function) Relationships: is_a GO:0016712 Definition: Catalysis of the reaction: (+)-costunolide (12,6alpha) + reduced [NADPH-hemoprotein reductase] + dioxygen = 3beta-hydroxycostunolide + oxidized [NADPH-hemoprotein reductase] + H2O. Sources: MetaCyc:RXN-15533